negative regulation of conidiophore development [GO:0070794] (biological process) Sources: GOC:mah Relationships: is_a regulation of conidiophore development [GO:0070793]; is_a negative regulation of spore-bearing organ development [GO:0075262]; negatively regulates conidiophore development [GO:0070787] Definition: Any process that stops, prevents, or reduces the frequency, rate or extent of conidiophore development, a process that leads to the formation of a conidiophore. The conidiophore is a specialized hypha that extends aerially from the growth substrate and bears conidia, or asexual spores. Subtypes: negative regulation of phialide development [GO:0070806]